venom-mediated perturbation of calcium channel activity [GO:0044472] (biological process) Relationships: is a type of venom-mediated perturbation of ion channel activity [GO:0044560] Definition: A process in which an organism alters or subverts the activity of a calcium channel in another organism via the action of a venom. Also known as: envenomation resulting in modulation of calcium channel activity in another organism, envenomation resulting in modulation of calcium channel activity in other organism Subtypes: GO:0044473 References: PMID:20920515 Sources: GOC:fj, GOC:jl